{
  "gene_name": "Atlastin-2",
  "gene": "UniProtKB:Q8NHH9",
  "term_id": "GO:0005525",
  "gene_symbol": "ATL2",
  "term_label": "GTP binding"
}